{
  "gene_symbol": "HTR7",
  "gene": "UniProtKB:P34969",
  "term_id": "GO:0030425",
  "gene_name": "5-hydroxytryptamine receptor 7",
  "term_label": "dendrite"
}